{
  "term_id": "GO:0045944",
  "gene_name": "Oxysterols receptor LXR-beta",
  "term_label": "positive regulation of transcription by RNA polymerase II",
  "gene_symbol": "NR1H2",
  "gene": "UniProtKB:P55055"
}